{
  "term_label": "plasma membrane",
  "gene": "UniProtKB:O00241",
  "gene_symbol": "SIRPB1",
  "term_id": "GO:0005886",
  "gene_name": "Signal-regulatory protein beta-1"
}